{
  "gene": "UniProtKB:P07438",
  "term_id": "GO:0005737",
  "gene_symbol": "MT1B",
  "gene_name": "Metallothionein-1B",
  "term_label": "cytoplasm"
}